{
  "term_id": "GO:0030511",
  "gene_symbol": "FLCN",
  "term_label": "positive regulation of transforming growth factor beta receptor signaling pathway",
  "gene": "UniProtKB:Q8NFG4",
  "gene_name": "Folliculin"
}